{
  "gene_symbol": "SCRT1",
  "term_id": "GO:0006355",
  "gene_name": "Transcriptional repressor scratch 1",
  "gene": "UniProtKB:Q9BWW7",
  "term_label": "regulation of DNA-templated transcription"
}